{
  "term_id": "UNKNOWN:0001",
  "term_label": "Unknown molecular function",
  "gene_name": "Putative nuclear receptor corepressor 1-like protein NCOR1P1",
  "gene": "UniProtKB:Q9H4R4",
  "gene_symbol": "NCOR1P1"
}